{
  "gene_name": "Golgin subfamily A member 6-like protein 6",
  "gene_symbol": "GOLGA6L6",
  "term_label": "Unknown biological process",
  "term_id": "UNKNOWN:0002",
  "gene": "UniProtKB:A8MZA4"
}